{
  "gene_symbol": "STXBP2",
  "gene": "UniProtKB:Q15833",
  "gene_name": "Syntaxin-binding protein 2",
  "term_label": "presynaptic dense core vesicle exocytosis",
  "term_id": "GO:0099525"
}